{
  "gene_symbol": "CACNG4",
  "gene_name": "Voltage-dependent calcium channel gamma-4 subunit",
  "term_label": "voltage-gated calcium channel activity",
  "term_id": "GO:0005245",
  "gene": "UniProtKB:Q9UBN1"
}